6,7-dihydropteridine reductase activity [GO:0004155] (molecular function) Relationships: is a type of oxidoreductase activity, acting on the CH-NH group of donors, NAD or NADP as acceptor [GO:0016646] Sources: EC:1.5.1.34 Also known as: dihydropteridine reductase activity, 5,6,7,8-tetrahydropteridine:NAD(P)+ oxidoreductase activity, 5,6,7,8-tetrahydropteridine:NAD(P)H+ oxidoreductase activity, 6,7-dihydropteridine:NAD(P)H oxidoreductase activity, DHPR activity, NAD(P)H(2):6,7-dihydropteridine oxidoreductase activity, NAD(P)H2:6,7-dihydropteridine oxidoreductase activity, NADH-dihydropteridine reductase activity, NADPH-dihydropteridine reductase activity, NADPH-specific dihydropteridine reductase activity, dihydropteridine (reduced nicotinamide adenine dinucleotide) reductase activity, dihydropteridine reductase (NADH) activity, dihydropteridine reduction Definition: Catalysis of the reaction: NAD(P)+ + 5,6,7,8-tetrahydropteridine = NAD(P)H + H+ + 6,7-dihydropteridine.